{
  "gene": "UniProtKB:Q92611",
  "gene_name": "ER degradation-enhancing alpha-mannosidase-like protein 1",
  "term_id": "UNKNOWN:0002",
  "gene_symbol": "EDEM1",
  "term_label": "Unknown biological process"
}